{
  "term_label": "Unknown cellular component",
  "gene_symbol": "GAL3ST3",
  "gene": "UniProtKB:Q96A11",
  "term_id": "UNKNOWN:0003",
  "gene_name": "Galactose-3-O-sulfotransferase 3"
}